positive regulation of skeletal muscle cell proliferation [GO:0014858] (biological process) Definition: Any process that activates or increases the frequency, rate or extent of skeletal muscle cell proliferation. Subtypes: GO:1902724 Sources: CL:0000188, GOC:ef, GOC:mtg_muscle Relationships: is a type of positive regulation of cell population proliferation [GO:0008284]; is a type of regulation of skeletal muscle cell proliferation [GO:0014857]; positively regulates GO:0014856